transcription factor TFIIIB-alpha complex [GO:0034732] (cellular component) References: PMID:11433012 Definition: A transcription factor TFIIIB-beta complex that contains the TATA-binding protein (TBP), B'' and a specialized homolog of the conserved subunit BRF referred to as BRFU or TFIIIB50, which found in human but not conserved in yeast; the complex is involved in the regulation of transcription from type 3 (upstream) RNA polymerase III promoters. Relationships: is a type of transcription factor TFIIIB complex [GO:0000126]